{
  "gene_symbol": "ANAPC10",
  "gene_name": "Anaphase-promoting complex subunit 10",
  "gene": "UniProtKB:Q9UM13",
  "term_label": "protein K11-linked ubiquitination",
  "term_id": "GO:0070979"
}